{
  "term_label": "spermatid development",
  "gene_symbol": "SEC23IP",
  "gene_name": "SEC23-interacting protein",
  "gene": "UniProtKB:Q9Y6Y8",
  "term_id": "GO:0007286"
}